{
  "term_id": "GO:0007155",
  "gene_symbol": "PCDH20",
  "term_label": "cell adhesion",
  "gene_name": "Protocadherin-20",
  "gene": "UniProtKB:Q8N6Y1"
}